regulation of macrophage antigen processing and presentation [GO:0002616] (BP) Relationships: is a type of regulation of antigen processing and presentation [GO:0002577]; regulates macrophage antigen processing and presentation [GO:0002472] Subtypes: negative regulation of macrophage antigen processing and presentation [GO:0002617], positive regulation of macrophage antigen processing and presentation [GO:0002618] Definition: Any process that modulates the frequency, rate, or extent of macrophage antigen processing and presentation. Sources: GOC:add